{
  "gene_symbol": "DHX36",
  "term_id": "GO:0002151",
  "gene_name": "ATP-dependent DNA_RNA helicase DHX36",
  "gene": "UniProtKB:Q9H2U1",
  "term_label": "G-quadruplex RNA binding"
}